[formate-C-acetyltransferase]-activating enzyme activity [GO:0043365] (molecular function) Relationships: is a type of glycyl-radical enzyme activating activity [GO:0043364] References: PMID:18307109 Sources: EC:1.97.1.4, GOC:jl Definition: Catalysis of the reaction: S-adenosyl-L-methionine + dihydroflavodoxin + [formate C-acetyltransferase]-glycine = 5'-deoxyadenosine + L-methionine + flavodoxin semiquinone + [formate C-acetyltransferase]-glycin-2-yl radical. Also known as: PFL activase activity, PFL-glycine:S-adenosyl-L-methionine H transferase (flavodoxin-oxidizing, S-adenosyl-L-methionine-cleaving) activity, [pyruvate formate-lyase]-activating enzyme activity, formate C-acetyltransferase-glycine dihydroflavodoxin:S-adenosyl-L-methionine oxidoreductase (S-adenosyl-L-methionine cleaving), formate acetyltransferase activating enzyme activity, formate acetyltransferase-glycine dihydroflavodoxin:S-adenosyl-L-methionine oxidoreductase (S-adenosyl-L-methionine cleaving) activity, formate-C-acetyltransferase-activating enzyme, pyruvate formate-lyase-activating enzyme